{
  "gene_symbol": "DMRT3",
  "gene_name": "Doublesex- and mab-3-related transcription factor 3",
  "term_label": "nucleus",
  "gene": "UniProtKB:Q9NQL9",
  "term_id": "GO:0005634"
}